{
  "gene": "UniProtKB:A0A087WWU0",
  "gene_symbol": "A0A087WWU0",
  "term_id": "UNKNOWN:0002",
  "gene_name": "Uncharacterized protein (Fragment)",
  "term_label": "Unknown biological process"
}